biphenyl metabolic process [GO:0018879] (biological process) Definition: The chemical reactions and pathways involving biphenyl, a toxic aromatic hydrocarbon used as a heat transfer agent, as a fungistat in packaging citrus fruits and in plant disease control. Biphenyl can be chlorinated with 1-10 chlorine molecules to form polychlorinated biphenyls (PCBs). Sources: GOC:jl Also known as: biphenyl metabolism, xenene metabolic process, xenene metabolism Relationships: is a type of benzene-containing compound metabolic process [GO:0042537] Subtypes: biphenyl catabolic process [GO:0070980]